{
  "term_label": "dynein heavy chain binding",
  "gene_name": "Cytoplasmic dynein 1 light intermediate chain 2",
  "term_id": "GO:0045504",
  "gene": "UniProtKB:O43237",
  "gene_symbol": "DYNC1LI2"
}